{
  "gene_symbol": "SETD2",
  "term_label": "regulation of gene expression",
  "gene_name": "Histone-lysine N-methyltransferase SETD2",
  "term_id": "GO:0010468",
  "gene": "UniProtKB:Q9BYW2"
}